skeletal muscle satellite cell fate determination [GO:0014818] (biological process) References: PMID:16607119 Sources: GOC:ef, GOC:mtg_muscle Definition: The process in which a cell becomes capable of differentiating autonomously into a skeletal muscle satellite cell regardless of its environment; upon determination, the cell fate cannot be reversed. Relationships: is a type of GO:0048867; is part of GO:0014813